intine [GO:0043678] (cellular component) Definition: The innermost of the major layers of the pollen grain wall which underlies the exine and borders the cytoplasm. References: PMID:33706055 Note: Note that the intine is not acetolysis resistant and is therefore absent in conventionally prepared palynological material. Relationships: is a type of cellular anatomical structure [GO:0110165]; BFO_0000050 GO:0043667